negative regulation of intestinal absorption [GO:1904479] (biological process) Relationships: is a type of negative regulation of digestive system process [GO:0060457]; is a type of regulation of intestinal absorption [GO:1904478]; negatively regulates GO:0050892 References: PMID:12469120 Sources: GOC:BHF, GOC:TermGenie, GOC:rl, GO_REF:0000058 Subtypes: GO:1904730 Definition: Any process that stops, prevents or reduces the frequency, rate or extent of intestinal absorption. Also known as: down regulation of intestinal absorption, down-regulation of intestinal absorption, downregulation of intestinal absorption, inhibition of intestinal absorption